{
  "gene_symbol": "CHMP6",
  "gene_name": "Charged multivesicular body protein 6",
  "gene": "UniProtKB:Q96FZ7",
  "term_label": "nuclear membrane reassembly",
  "term_id": "GO:0031468"
}